ERBB signaling pathway [GO:0038127] (biological process) Relationships: is a type of cell surface receptor protein tyrosine kinase signaling pathway [GO:0007169] Subtypes: epidermal growth factor receptor signaling pathway [GO:0007173], GO:0038128, ERBB3 signaling pathway [GO:0038129], ERBB4 signaling pathway [GO:0038130] References: PMID:16460914 Sources: GOC:jc, Wikipedia:ErbB Also known as: EGF receptor family signaling pathway, ERBB signalling pathway, ErbB signaling, EGFR family signaling pathway Definition: The series of molecular signals initiated by binding of a ligand to a member of the ERBB family of receptor tyrosine kinases on the surface of a cell, and ending with the regulation of a downstream cellular process, e.g. transcription. Regulation: RO_0002211 by regulation of ERBB signaling pathway [GO:1901184]; negatively regulated by negative regulation of ERBB signaling pathway [GO:1901185]; positively regulated by positive regulation of ERBB signaling pathway [GO:1901186]